{
  "term_id": "GO:0098978",
  "gene": "UniProtKB:Q9ULU8",
  "gene_name": "Calcium-dependent secretion activator 1",
  "gene_symbol": "CADPS",
  "term_label": "glutamatergic synapse"
}